{
  "term_label": "plasma membrane",
  "term_id": "GO:0005886",
  "gene_name": "Inward rectifier potassium channel 4",
  "gene_symbol": "KCNJ4",
  "gene": "UniProtKB:P48050"
}